stachyose synthase activity [GO:0102831] (molecular function) Relationships: is a type of hexosyltransferase activity [GO:0016758] References: PMID:12060258 Sources: GOC:pz Definition: Catalysis of the reaction: 2 raffinose = stachyose + sucrose.